{
  "term_label": "peptide antigen assembly with MHC class II protein complex",
  "term_id": "GO:0002503",
  "gene": "UniProtKB:P01920",
  "gene_symbol": "HLA-DQB1",
  "gene_name": "HLA class II histocompatibility antigen, DQ beta 1 chain"
}